{
  "term_id": "GO:0007165",
  "gene": "UniProtKB:P28827",
  "gene_name": "Receptor-type tyrosine-protein phosphatase mu",
  "gene_symbol": "PTPRM",
  "term_label": "signal transduction"
}